{
  "gene": "UniProtKB:Q9Y580",
  "term_id": "GO:0003727",
  "gene_name": "RNA-binding protein 7",
  "gene_symbol": "RBM7",
  "term_label": "single-stranded RNA binding"
}